{
  "term_id": "GO:0005509",
  "term_label": "calcium ion binding",
  "gene_symbol": "KCNIP4",
  "gene_name": "Kv channel-interacting protein 4",
  "gene": "UniProtKB:Q6PIL6"
}